{
  "term_id": "GO:0005886",
  "term_label": "plasma membrane",
  "gene_symbol": "ARHGEF40",
  "gene_name": "Rho guanine nucleotide exchange factor 40",
  "gene": "UniProtKB:Q8TER5"
}